exocytic insertion of neurotransmitter receptor to plasma membrane [GO:0098881] (biological process) References: PMID:19503082 Sources: GOC:aruk, GOC:bc Definition: The exocytic fusion of neurotransmitter receptor-containing vesicles with plasma membrane, resulting in the integration of neurotransmitter receptors into the plasma membrane. This process includes tethering and docking steps that prepare vesicles for fusion. Also known as: neurotransmitter receptor insertion Relationships: is a type of vesicle docking involved in exocytosis [GO:0006904]; is a type of GO:0090522; BFO_0000050 GO:0098877